{
  "term_id": "GO:0035459",
  "gene_name": "Uncharacterized protein",
  "gene": "UniProtKB:A0A2R8YE69",
  "term_label": "vesicle cargo loading",
  "gene_symbol": "A0A2R8YE69"
}